G protein-coupled receptor signaling pathway involved in social behavior [GO:1904068] (biological process) Definition: Any G protein-coupled receptor signaling pathway that is involved in social behavior. References: PMID:22665789 Sources: GOC:TermGenie, GOC:kmv, GO_REF:0000060 Also known as: G protein coupled receptor protein signaling pathway involved in social behavior, G protein coupled receptor protein signaling pathway involved in social behaviour, G protein coupled receptor protein signalling pathway involved in social behavior, G protein coupled receptor protein signalling pathway involved in social behaviour, G-protein coupled receptor protein signal transduction involved in social behavior, G-protein coupled receptor protein signal transduction involved in social behaviour, G-protein coupled receptor protein signaling pathway involved in social behavior, G-protein coupled receptor protein signaling pathway involved in social behaviour, G-protein coupled receptor signaling pathway involved in social behavior, G-protein coupled receptor signaling pathway involved in social behaviour, G-protein coupled receptor signalling pathway involved in social behavior, G-protein coupled receptor signalling pathway involved in social behaviour, G-protein-coupled receptor protein signaling pathway involved in social behavior, G-protein-coupled receptor protein signaling pathway involved in social behaviour, G-protein-coupled receptor protein signalling pathway involved in social behavior, G-protein-coupled receptor protein signalling pathway involved in social behaviour, GPCR signaling pathway involved in social behavior, GPCR signaling pathway involved in social behaviour, GPCR signalling pathway involved in social behavior, GPCR signalling pathway involved in social behaviour, G protein coupled receptor protein signaling pathway involved in cooperative behavior, G protein coupled receptor protein signalling pathway involved in cooperative behavior, G-protein coupled receptor protein signal transduction involved in cooperative behavior, G-protein coupled receptor protein signaling pathway involved in cooperative behavior, G-protein coupled receptor signaling pathway involved in cooperative behavior, G-protein coupled receptor signalling pathway involved in cooperative behavior, G-protein-coupled receptor protein signaling pathway involved in cooperative behavior, G-protein-coupled receptor protein signalling pathway involved in cooperative behavior, GPCR signaling pathway involved in cooperative behavior, GPCR signalling pathway involved in cooperative behavior Relationships: is a type of GO:0007186; is part of GO:0035176